DNA-dependent protein kinase-DNA ligase 4 complex [GO:0005958] (cellular component) References: PMID:10854421, PMID:12235392, PMID:17072889 Sources: GOC:jl, GOC:mah Definition: A large protein complex which is involved in the repair of DNA double-strand breaks and, in mammals, V(D)J recombination events. It consists of the DNA-dependent protein kinase catalytic subunit (DNA-PKcs), the DNA end-binding heterodimer Ku, the nuclear phosphoprotein XRCC4 or a homolog thereof, and DNA ligase IV. Relationships: is a type of nonhomologous end joining complex [GO:0070419]; is a type of nuclear protein-containing complex [GO:0140513]